regulation of collagen metabolic process [GO:0010712] (biological process) Definition: Any process that modulates the frequency, rate or extent of the chemical reactions and pathways resulting in the metabolism of collagen, any of a group of fibrous proteins of very high tensile strength that form the main component of connective tissue in animals. Sources: GOC:dph, GOC:tb Also known as: regulation of collagen metabolism Subtypes: regulation of collagen catabolic process [GO:0010710], negative regulation of collagen metabolic process [GO:0010713], positive regulation of collagen metabolic process [GO:0010714], GO:0032965 Relationships: is_a GO:0019222; regulates collagen metabolic process [GO:0032963]